{
  "term_id": "UNKNOWN:0002",
  "gene_symbol": "MED13L",
  "gene_name": "Mediator of RNA polymerase II transcription subunit 13-like",
  "term_label": "Unknown biological process",
  "gene": "UniProtKB:Q71F56"
}